{
  "term_label": "protein serine/threonine kinase activity",
  "gene_name": "Serine_threonine-protein kinase ULK2",
  "term_id": "GO:0004674",
  "gene_symbol": "ULK2",
  "gene": "UniProtKB:Q8IYT8"
}